{
  "gene_name": "Arylacetamide deacetylase-like 4",
  "gene_symbol": "AADACL4",
  "term_label": "Unknown biological process",
  "term_id": "UNKNOWN:0002",
  "gene": "UniProtKB:Q5VUY2"
}